{
  "term_label": "glutathione biosynthetic process",
  "gene_name": "Glutamate--cysteine ligase catalytic subunit",
  "gene": "UniProtKB:P48506",
  "gene_symbol": "GCLC",
  "term_id": "GO:0006750"
}